{
  "gene_symbol": "PPP2R1A",
  "term_id": "GO:0051754",
  "term_label": "meiotic sister chromatid cohesion, centromeric",
  "gene": "UniProtKB:P30153",
  "gene_name": "Serine_threonine-protein phosphatase 2A 65 kDa regulatory subunit A alpha isoform"
}